{
  "term_label": "Unknown biological process",
  "term_id": "UNKNOWN:0002",
  "gene": "UniProtKB:Q96L46",
  "gene_symbol": "CAPNS2",
  "gene_name": "Calpain small subunit 2"
}